{
  "term_id": "GO:0005930",
  "gene_name": "Coiled-coil domain-containing protein 96",
  "gene_symbol": "CFAP184",
  "gene": "UniProtKB:Q2M329",
  "term_label": "axoneme"
}